{
  "gene": "UniProtKB:Q8TCT0",
  "gene_symbol": "CERK",
  "term_label": "plasma membrane",
  "gene_name": "Ceramide kinase",
  "term_id": "GO:0005886"
}